{
  "gene": "UniProtKB:Q01804",
  "term_id": "GO:0061578",
  "gene_name": "OTU domain-containing protein 4",
  "term_label": "K63-linked deubiquitinase activity",
  "gene_symbol": "OTUD4"
}